{
  "gene_name": "Kynurenine--oxoglutarate transaminase 3",
  "term_label": "Unknown biological process",
  "term_id": "UNKNOWN:0002",
  "gene": "UniProtKB:Q6YP21",
  "gene_symbol": "KYAT3"
}